AMPA selective glutamate receptor signaling pathway [GO:0098990] (biological process) Definition: The series of molecular signals initiated by glutamate binding to an AMPA-selective glutamate receptor on the surface of the target cell, followed by the movement of ions through a channel in the receptor complex, and ending with the regulation of a downstream cellular process, e.g. transcription. Relationships: is a type of GO:0035235; has part AMPA glutamate receptor activity [GO:0004971] Sources: GOC:dos, ISBN:9780071120005